{
  "term_label": "mitochondrion",
  "gene_name": "Mitochondrial genome maintenance exonuclease 1",
  "gene_symbol": "MGME1",
  "gene": "UniProtKB:Q9BQP7",
  "term_id": "GO:0005739"
}